negative regulation of nuclear cell cycle DNA replication [GO:1902576] (biological process) References: PMID:19033384 Sources: GOC:TermGenie Relationships: is a type of negative regulation of cell cycle process [GO:0010948]; is a type of regulation of nuclear cell cycle DNA replication [GO:0033262]; is a type of negative regulation of DNA-templated DNA replication [GO:2000104]; RO_0002212 nuclear DNA replication [GO:0033260] Definition: Any process that stops, prevents or reduces the frequency, rate or extent of nuclear cell cycle DNA replication. Subtypes: negative regulation of mitotic cell cycle DNA replication [GO:1903464], negative regulation of initiation of premeiotic DNA replication [GO:1904513] Also known as: down regulation of DNA replication involved in S phase, down regulation of DNA replication involved in S-phase, down regulation of nuclear cell cycle DNA replication, down-regulation of DNA replication involved in S phase, down-regulation of DNA replication involved in S-phase, down-regulation of nuclear cell cycle DNA replication, downregulation of DNA replication involved in S phase, downregulation of DNA replication involved in S-phase, downregulation of nuclear cell cycle DNA replication, negative regulation of DNA replication involved in S phase, negative regulation of DNA replication involved in S-phase, inhibition of DNA replication involved in S phase, inhibition of DNA replication involved in S-phase, inhibition of nuclear cell cycle DNA replication, down regulation of DNA replication during S phase, down-regulation of DNA replication during S phase, downregulation of DNA replication during S phase, inhibition of DNA replication during S phase, negative regulation of DNA replication during S phase